{
  "gene_symbol": "TRPC5OS",
  "term_label": "Unknown molecular function",
  "term_id": "UNKNOWN:0001",
  "gene": "UniProtKB:A6NMA1",
  "gene_name": "Putative uncharacterized protein TRPC5OS"
}